{
  "gene": "UniProtKB:Q96A00",
  "term_label": "Unknown cellular component",
  "term_id": "UNKNOWN:0003",
  "gene_symbol": "PPP1R14A",
  "gene_name": "Protein phosphatase 1 regulatory subunit 14A"
}